regulation of gonadotropin secretion [GO:0032276] (BP) Subtypes: negative regulation of gonadotropin secretion [GO:0032277], positive regulation of gonadotropin secretion [GO:0032278], regulation of luteinizing hormone secretion [GO:0033684], GO:0046880 Sources: GOC:mah Relationships: is a type of regulation of endocrine process [GO:0044060]; is a type of regulation of hormone secretion [GO:0046883]; regulates GO:0032274 Definition: Any process that modulates the frequency, rate or extent of the regulated release of a gonadotropin. Also known as: regulation of gonadotrophin secretion